{
  "gene": "UniProtKB:O96014",
  "term_label": "cell fate commitment",
  "gene_symbol": "WNT11",
  "term_id": "GO:0045165",
  "gene_name": "Protein Wnt-11"
}